SCAR complex [GO:0031209] (cellular component) Also known as: WRC, WAVE complex, WAVE regulatory complex References: PMID:12181570, PMID:24036345, PMID:24630101 Sources: GOC:hla, GOC:pg Definition: A pentameric complex that includes orthologues of human PIR121, Nap1, Abi, SCAR, and HSPC300 and regulates actin polymerization and/or depolymerization through small GTPase mediated signal transduction. Relationships: is a type of protein-containing complex [GO:0032991]; is part of cytoplasm [GO:0005737]